{
  "gene": "UniProtKB:P55786",
  "term_id": "GO:0070006",
  "gene_name": "Puromycin-sensitive aminopeptidase",
  "term_label": "metalloaminopeptidase activity",
  "gene_symbol": "NPEPPS"
}